{
  "gene": "UniProtKB:O00142",
  "term_label": "mitochondrion",
  "term_id": "GO:0005739",
  "gene_symbol": "TK2",
  "gene_name": "Thymidine kinase 2, mitochondrial"
}